{
  "term_label": "palmitoyl-CoA 9-desaturase activity",
  "gene": "UniProtKB:O00767",
  "gene_symbol": "SCD",
  "term_id": "GO:0032896",
  "gene_name": "Stearoyl-CoA desaturase"
}